{
  "gene_symbol": "MDP1",
  "gene_name": "Magnesium-dependent phosphatase 1",
  "gene": "UniProtKB:Q86V88",
  "term_id": "UNKNOWN:0003",
  "term_label": "Unknown cellular component"
}